{
  "term_label": "vesicle-mediated transport",
  "gene_name": "Vacuolar fusion protein CCZ1 homolog",
  "gene_symbol": "CCZ1",
  "term_id": "GO:0016192",
  "gene": "UniProtKB:P86791"
}